{
  "term_id": "GO:0031468",
  "gene": "UniProtKB:P68543",
  "gene_name": "UBX domain-containing protein 2A",
  "gene_symbol": "UBXN2A",
  "term_label": "nuclear membrane reassembly"
}